{
  "gene": "UniProtKB:O75570",
  "gene_name": "Peptide chain release factor 1, mitochondrial",
  "term_label": "mitochondrial translational termination",
  "gene_symbol": "MTRF1",
  "term_id": "GO:0070126"
}